{
  "term_id": "GO:0007420",
  "gene_symbol": "SOX2",
  "term_label": "brain development",
  "gene_name": "Transcription factor SOX-2",
  "gene": "UniProtKB:P48431"
}